{
  "gene": "UniProtKB:Q9H4A9",
  "term_label": "dipeptidase activity",
  "gene_symbol": "DPEP2",
  "gene_name": "Dipeptidase 2",
  "term_id": "GO:0016805"
}